{
  "gene": "UniProtKB:P78346",
  "gene_name": "Ribonuclease P protein subunit p30",
  "term_id": "GO:0005655",
  "term_label": "nucleolar ribonuclease P complex",
  "gene_symbol": "RPP30"
}